{
  "gene_name": "Unconventional myosin-Ia",
  "term_id": "GO:0000146",
  "gene_symbol": "MYO1A",
  "term_label": "microfilament motor activity",
  "gene": "UniProtKB:Q9UBC5"
}